{
  "gene_name": "Olfactory receptor 6C74",
  "gene_symbol": "OR6C74",
  "gene": "UniProtKB:A6NCV1",
  "term_id": "GO:0005886",
  "term_label": "plasma membrane"
}